{
  "term_id": "GO:0002682",
  "gene_symbol": "ZBTB37",
  "term_label": "regulation of immune system process",
  "gene_name": "Zinc finger and BTB domain-containing protein 37",
  "gene": "UniProtKB:Q5TC79"
}